{
  "gene_name": "Insulin-like growth factor I",
  "term_label": "negative regulation of apoptotic process",
  "term_id": "GO:0043066",
  "gene_symbol": "IGF1",
  "gene": "UniProtKB:P05019"
}